{
  "gene": "UniProtKB:Q8TC21",
  "gene_symbol": "ZNF596",
  "term_label": "nucleus",
  "term_id": "GO:0005634",
  "gene_name": "Zinc finger protein 596"
}